{
  "gene_symbol": "CIST1",
  "term_label": "Unknown cellular component",
  "term_id": "UNKNOWN:0003",
  "gene": "UniProtKB:A0A2R8Y7Y5",
  "gene_name": "Protein CIST1"
}